{
  "term_label": "telomere maintenance",
  "gene_symbol": "ATR",
  "term_id": "GO:0000723",
  "gene_name": "Serine_threonine-protein kinase ATR",
  "gene": "UniProtKB:Q13535"
}